structural constituent of postsynaptic actin cytoskeleton [GO:0098973] (MF) Definition: The action of a molecule that contributes to the structural integrity of a postsynaptic actin cytoskeleton. Sources: GOC:dos Relationships: is a type of structural constituent of cytoskeleton [GO:0005200]; is a type of structural constituent of postsynapse [GO:0099186]; is part of postsynaptic actin cytoskeleton organization [GO:0098974]; occurs in postsynaptic actin cytoskeleton [GO:0098871]